{
  "gene_symbol": "ST6GALNAC2",
  "term_label": "protein O-linked glycosylation",
  "term_id": "GO:0006493",
  "gene_name": "Alpha-N-acetylgalactosaminide alpha-2,6-sialyltransferase 2",
  "gene": "UniProtKB:Q9UJ37"
}